{
  "gene_symbol": "GSDMB",
  "gene_name": "Gasdermin-B",
  "gene": "UniProtKB:Q8TAX9",
  "term_id": "GO:0005546",
  "term_label": "phosphatidylinositol-4,5-bisphosphate binding"
}